{
  "gene": "UniProtKB:Q9C040",
  "term_label": "proteasome-mediated ubiquitin-dependent protein catabolic process",
  "gene_symbol": "TRIM2",
  "gene_name": "Tripartite motif-containing protein 2",
  "term_id": "GO:0043161"
}